{
  "term_label": "RNA polymerase II cis-regulatory region sequence-specific DNA binding",
  "gene": "UniProtKB:P35713",
  "term_id": "GO:0000978",
  "gene_name": "Transcription factor SOX-18",
  "gene_symbol": "SOX18"
}